negative regulation of melanosome transport [GO:1902909] (biological process) Relationships: is a type of GO:0048523; is a type of negative regulation of transport [GO:0051051]; is a type of regulation of melanosome transport [GO:1902908]; negatively regulates GO:0032402 References: PMID:23334344 Sources: GOC:TermGenie, GOC:als, GO_REF:0000058 Definition: Any process that stops, prevents or reduces the frequency, rate or extent of melanosome transport. Also known as: down regulation of melanosome transport, down-regulation of melanosome transport, downregulation of melanosome transport, inhibition of melanosome transport